{
  "term_id": "GO:0005737",
  "gene_name": "Tyrosine-protein phosphatase non-receptor type 4",
  "term_label": "cytoplasm",
  "gene_symbol": "PTPN4",
  "gene": "UniProtKB:P29074"
}